{
  "term_id": "GO:0050650",
  "term_label": "chondroitin sulfate proteoglycan biosynthetic process",
  "gene": "UniProtKB:Q9P2W7",
  "gene_name": "Galactosylgalactosylxylosylprotein 3-beta-glucuronosyltransferase 1",
  "gene_symbol": "B3GAT1"
}